regulation of T cell apoptotic process [GO:0070232] (biological process) Relationships: is a type of regulation of lymphocyte apoptotic process [GO:0070228]; regulates T cell apoptotic process [GO:0070231] Sources: GOC:add, GOC:mtg_apoptosis, ISBN:0781765196 Definition: Any process that modulates the occurrence or rate of T cell death by apoptotic process. Subtypes: GO:0070233, positive regulation of T cell apoptotic process [GO:0070234], GO:0070235, GO:0070239, regulation of thymocyte apoptotic process [GO:0070243], regulation of activated CD4-positive, alpha-beta T cell apoptotic process [GO:1905399], GO:1905402 Also known as: regulation of T lymphocyte apoptosis, regulation of T-cell apoptosis, regulation of T-lymphocyte apoptosis, regulation of programmed cell death of T cells by apoptosis, regulation of T cell apoptosis